{
  "gene": "UniProtKB:Q3B7T3",
  "gene_symbol": "BEAN1",
  "term_id": "UNKNOWN:0001",
  "term_label": "Unknown molecular function",
  "gene_name": "Protein BEAN1"
}